{
  "gene": "UniProtKB:Q16600",
  "term_label": "RNA polymerase II cis-regulatory region sequence-specific DNA binding",
  "term_id": "GO:0000978",
  "gene_symbol": "ZNF239",
  "gene_name": "Zinc finger protein 239"
}